{
  "gene": "UniProtKB:Q9UBP0",
  "term_label": "ATP hydrolysis activity",
  "gene_name": "Spastin",
  "term_id": "GO:0016887",
  "gene_symbol": "SPAST"
}